{
  "term_label": "nucleolus",
  "gene_symbol": "CCDC86",
  "term_id": "GO:0005730",
  "gene": "UniProtKB:Q9H6F5",
  "gene_name": "Coiled-coil domain-containing protein 86"
}